sterol 24-C-methyltransferase activity [GO:0003838] (MF) Relationships: is a type of C-methyltransferase activity [GO:0008169]; is a type of S-adenosylmethionine-dependent methyltransferase activity [GO:0008757] Sources: RHEA:21128 Also known as: delta(24)-sterol C-methyltransferase activity, sterol 24C methyltransferase activity, SMT1 activity, phytosterol methyltransferase activity, zymosterol-24-methyltransferase activity, 24-sterol C-methyltransferase activity, S-adenosyl-4-methionine:sterol Delta(24)-methyltransferase activity, S-adenosyl-4-methionine:sterol delta24-methyltransferase activity, S-adenosyl-L-methionine:Delta(24(23))-sterol methyltransferase activity, S-adenosyl-L-methionine:Delta24(23)-sterol methyltransferase activity, S-adenosyl-L-methionine:zymosterol 24-C-methyltransferase activity, delta(24)-methyltransferase activity, delta(24)-sterol methyltransferase activity, delta24-methyltransferase activity, delta24-sterol methyltransferase activity Definition: Catalysis of the reaction: S-adenosyl-L-methionine + zymosterol = fecosterol + H+ + S-adenosyl-L-homocysteine.